{
  "gene": "UniProtKB:P12036",
  "gene_name": "Neurofilament heavy polypeptide",
  "gene_symbol": "NEFH",
  "term_id": "GO:0030424",
  "term_label": "axon"
}